{
  "gene_name": "Zinc finger protein 407",
  "gene_symbol": "ZNF407",
  "gene": "UniProtKB:Q9C0G0",
  "term_label": "DNA-binding transcription factor activity",
  "term_id": "GO:0003700"
}